{
  "gene_symbol": "GAS2",
  "gene": "UniProtKB:O43903",
  "gene_name": "Growth arrest-specific protein 2",
  "term_label": "Unknown cellular component",
  "term_id": "UNKNOWN:0003"
}